penetration of cumulus oophorus [GO:0061956] (biological process) Also known as: penetration of cumulus cells layer, penetration of cumulus mass Relationships: is a type of multicellular organismal reproductive process [GO:0048609]; is part of single fertilization [GO:0007338] Definition: The infiltration by sperm of the cumulus oophorus to reach the oocyte. The process involves digestive enzymes from a modified lysosome called the acrosome, situated at the head of the sperm. References: PMID:21380641